{
  "term_label": "Unknown molecular function",
  "gene_symbol": "ERVW-1",
  "term_id": "UNKNOWN:0001",
  "gene": "UniProtKB:Q9UQF0",
  "gene_name": "Syncytin-1"
}